{
  "term_label": "Unknown molecular function",
  "gene_symbol": "SPRR3",
  "gene": "UniProtKB:Q9UBC9",
  "term_id": "UNKNOWN:0001",
  "gene_name": "Small proline-rich protein 3"
}